cysteine transport [GO:0042883] (biological process) Relationships: is a type of sulfur amino acid transport [GO:0000101]; is a type of organic cation transport [GO:0015695]; is a type of neutral amino acid transport [GO:0015804] Subtypes: GO:1903712 Also known as: L-cysteine transport Sources: GOC:jl, ISBN:0198506732 Definition: The directed movement of cysteine into, out of or within a cell, or between cells, by means of some agent such as a transporter or pore.